positive regulation of adenylate cyclase-inhibiting dopamine receptor signaling pathway [GO:1904992] (biological process) Relationships: is a type of positive regulation of dopamine receptor signaling pathway [GO:0060161]; is a type of regulation of adenylate cyclase-inhibiting dopamine receptor signaling pathway [GO:1904990]; positively regulates adenylate cyclase-inhibiting dopamine receptor signaling pathway [GO:0007195] References: PMID:26554819 Sources: GOC:TermGenie, GOC:kmv, GO_REF:0000058 Definition: Any process that activates or increases the frequency, rate or extent of adenylate cyclase-inhibiting dopamine receptor signaling pathway. Also known as: positive regulation of dopamine receptor, adenylate cyclase inhibiting pathway, positive regulation of dopamine receptor, adenylyl cyclase inhibiting pathway, positive regulation of inhibition of adenylate cyclase activity by dopamine receptor signalling pathway, up regulation of adenylate cyclase-inhibiting dopamine receptor signaling pathway, up regulation of dopamine receptor, adenylate cyclase inhibiting pathway, up regulation of dopamine receptor, adenylyl cyclase inhibiting pathway, up regulation of inhibition of adenylate cyclase activity by dopamine receptor signalling pathway, up-regulation of adenylate cyclase-inhibiting dopamine receptor signaling pathway, up-regulation of dopamine receptor, adenylate cyclase inhibiting pathway, up-regulation of dopamine receptor, adenylyl cyclase inhibiting pathway, up-regulation of inhibition of adenylate cyclase activity by dopamine receptor signalling pathway, upregulation of adenylate cyclase-inhibiting dopamine receptor signaling pathway, upregulation of dopamine receptor, adenylate cyclase inhibiting pathway, upregulation of dopamine receptor, adenylyl cyclase inhibiting pathway, upregulation of inhibition of adenylate cyclase activity by dopamine receptor signalling pathway, activation of adenylate cyclase-inhibiting dopamine receptor signaling pathway, activation of dopamine receptor, adenylate cyclase inhibiting pathway, activation of dopamine receptor, adenylyl cyclase inhibiting pathway, activation of inhibition of adenylate cyclase activity by dopamine receptor signalling pathway, activation of inhibition of adenylate cyclase activity by dopamine receptor signaling pathway, positive regulation of inhibition of adenylate cyclase activity by dopamine receptor signaling pathway, up regulation of inhibition of adenylate cyclase activity by dopamine receptor signaling pathway, up-regulation of inhibition of adenylate cyclase activity by dopamine receptor signaling pathway, upregulation of inhibition of adenylate cyclase activity by dopamine receptor signaling pathway